{
  "gene_symbol": "TMEM243",
  "gene_name": "Transmembrane protein 243",
  "gene": "UniProtKB:Q9BU79",
  "term_label": "Unknown cellular component",
  "term_id": "UNKNOWN:0003"
}